rRNA (adenine) methyltransferase activity [GO:0016433] (molecular function) Relationships: is a type of rRNA methyltransferase activity [GO:0008649] Definition: Catalysis of the reaction: S-adenosyl-L-methionine + rRNA = S-adenosyl-L-homocysteine + rRNA containing methyladenine. Sources: GOC:go-curators Subtypes: GO:0000179, rRNA (adenine-N6-)-methyltransferase activity [GO:0008988], 23S rRNA (adenosine(1067)-2'-O)-methyltransferase activity [GO:0030743], rRNA (adenine(2503)-C2-)-methyltransferase activity [GO:0070040], GO:0106142